{
  "gene_name": "3-oxoacyl-[acyl-carrier-protein] reductase",
  "term_label": "quinone binding",
  "gene": "UniProtKB:Q8N4T8",
  "gene_symbol": "CBR4",
  "term_id": "GO:0048038"
}